{
  "term_label": "Unknown cellular component",
  "term_id": "UNKNOWN:0003",
  "gene": "UniProtKB:Q8TBK6",
  "gene_name": "Zinc finger CCHC domain-containing protein 10",
  "gene_symbol": "ZCCHC10"
}